{
  "gene": "UniProtKB:P30530",
  "term_label": "plasma membrane",
  "gene_name": "Tyrosine-protein kinase receptor UFO",
  "gene_symbol": "AXL",
  "term_id": "GO:0005886"
}